septin ring [GO:0005940] (cellular component) Subtypes: cellular bud neck septin ring [GO:0000144], hyphal septin ring [GO:0032168], prospore septin ring [GO:0032169], pseudohyphal septin ring [GO:0032170], germ tube septin ring [GO:0032172], mating projection septin ring [GO:0032175], GO:0036391 Relationships: is a type of septin cytoskeleton [GO:0032156]; is part of cytoskeleton [GO:0005856]; is part of GO:0005938 References: PMID:16009555, PMID:16151244 Sources: GOC:krc, GOC:mah Definition: A tight ring-shaped structure that forms in the division plane at the site of cytokinesis; composed of members of the conserved family of filament-forming proteins called septins as well as septin-associated proteins. This type of septin structure is observed at the bud neck of budding fungal cells, at the site of cell division in animal cells, at the junction between the mother cell and a pseudohyphal projection, and also within hyphae of filamentous fungi at sites where a septum will form.